protein-N(PI)-phosphohistidine-N-acetyl-mannosamine phosphotransferase system transporter activity [GO:0090591] (molecular function) Relationships: is a type of GO:0008982 References: PMID:9864311 Definition: Catalysis of the PEP-dependent, phosphoryl transfer-driven transport of substances across a membrane. The transport happens by catalysis of the reaction: protein N-phosphohistidine + N-acetyl-mannosamine(out) = protein histidine +N-acetyl- mannosamine-6-phosphate(in).